{
  "term_id": "GO:0005886",
  "term_label": "plasma membrane",
  "gene_name": "Synaptotagmin-like protein 3",
  "gene_symbol": "SYTL3",
  "gene": "UniProtKB:Q4VX76"
}